{
  "gene": "UniProtKB:O75920",
  "term_id": "UNKNOWN:0002",
  "term_label": "Unknown biological process",
  "gene_symbol": "SERF1B",
  "gene_name": "Small EDRK-rich factor 1"
}